{
  "term_id": "UNKNOWN:0003",
  "gene_symbol": "FAM167B",
  "term_label": "Unknown cellular component",
  "gene_name": "Protein FAM167B",
  "gene": "UniProtKB:Q9BTA0"
}